{
  "gene_name": "Carbonyl reductase [NADPH] 3",
  "term_id": "UNKNOWN:0002",
  "gene_symbol": "CBR3",
  "gene": "UniProtKB:O75828",
  "term_label": "Unknown biological process"
}